negative regulation of acute inflammatory response [GO:0002674] (biological process) Sources: GOC:add Relationships: is a type of regulation of acute inflammatory response [GO:0002673]; is a type of GO:0050728; negatively regulates acute inflammatory response [GO:0002526] Also known as: down regulation of acute inflammatory response, down-regulation of acute inflammatory response, downregulation of acute inflammatory response, inhibition of acute inflammatory response Subtypes: GO:0002257, negative regulation of acute inflammatory response to antigenic stimulus [GO:0002865], negative regulation of acute inflammatory response to non-antigenic stimulus [GO:0002878], GO:0031621 Definition: Any process that stops, prevents, or reduces the frequency, rate, or extent of an acute inflammatory response.